clathrin coating of Golgi vesicle, trans-Golgi to endosome targeting [GO:0010786] (biological process) Definition: The addition of clathrin and adaptor proteins to Golgi membranes during the formation of transport vesicles that will move from the trans-Golgi to the endosome, forming a vesicle coat. Relationships: is a type of GO:0048202; is part of vesicle targeting, trans-Golgi to endosome [GO:0048203] Sources: GOC:dph, GOC:tb